5-n-alk(en)ylresorcinol O-methyltransferase activity [GO:0102990] (molecular function) Definition: Catalysis of the reaction: (8Z,11Z)-5-(pentadeca-8,11,14-trien-1-yl)resorcinol + S-adenosyl-L-methionine = (8Z,11Z)-5-(pentadeca- 8,11,14-trien-1-yl)resorcinol-3-methyl ether + H+ + S-adenosyl-L-homocysteine. Relationships: is a type of methyltransferase activity [GO:0008168] Sources: RHEA:26325